{
  "term_id": "UNKNOWN:0003",
  "term_label": "Unknown cellular component",
  "gene": "UniProtKB:Q8NB46",
  "gene_name": "Serine_threonine-protein phosphatase 6 regulatory ankyrin repeat subunit C",
  "gene_symbol": "ANKRD52"
}